dosage compensation by inactivation of X chromosome [GO:0009048] (BP) Subtypes: random inactivation of X chromosome [GO:0060816], GO:0060818 References: PMID:11498577, PMID:20622855 Sources: GOC:jl, GOC:mr, GOC:pr, Wikipedia:XY_sex-determination_system Also known as: chromosome inactivation, X chromosome inactivation, Barr body formation Definition: Compensating for the two-fold variation in X-chromosome:autosome ratios between sexes by heterochromatin formation leading to a global inactivation of all, or most of, the genes on one of the X-chromosomes in the XX sex. Relationships: is a type of sex-chromosome dosage compensation [GO:0007549]; is a type of heterochromatin formation [GO:0031507]